{
  "gene_symbol": "TREM2",
  "term_id": "GO:1903980",
  "term_label": "positive regulation of microglial cell activation",
  "gene": "UniProtKB:Q9NZC2",
  "gene_name": "Triggering receptor expressed on myeloid cells 2"
}